fucose-1-phosphate guanylyltransferase activity [GO:0047341] (molecular function) Relationships: is a type of guanylyltransferase activity [GO:0070568] Sources: RHEA:13549 Also known as: GTP:fucose-1-phosphate guanylyltransferase activity, GDP fucose pyrophosphorylase activity, GDP-L-fucose pyrophosphorylase activity, GDP-fucose diphosphorylase activity, GDP-fucose pyrophosphorylase activity, GTP:L-fucose-1-phosphate guanylyltransferase activity, GTP:beta-L-fucose-1-phosphate guanylyltransferase activity, guanosine diphosphate L-fucose pyrophosphorylase activity Definition: Catalysis of the reaction: beta-L-fucose 1-phosphate + GTP + H+ = diphosphate + GDP-beta-L-fucose.